{
  "gene_name": "Large ribosomal subunit protein mL65",
  "gene": "UniProtKB:Q9NP92",
  "gene_symbol": "MRPS30",
  "term_id": "GO:0005762",
  "term_label": "mitochondrial large ribosomal subunit"
}